uronate dehydrogenase activity [GO:0050388] (molecular function) Also known as: uronate: NAD-oxidoreductase activity, uronate:NAD+ 1-oxidoreductase activity, uronic acid dehydrogenase activity Sources: EC:1.1.1.203, RHEA:22404 Definition: Catalysis of the reaction: D-galacturonate + H2O + NAD+ = galactarate + 2 H+ + NADH. Relationships: is a type of oxidoreductase activity, acting on the CH-OH group of donors, NAD or NADP as acceptor [GO:0016616]